{
  "gene_symbol": "CNTNAP1",
  "term_label": "myelination",
  "gene": "UniProtKB:P78357",
  "gene_name": "Contactin-associated protein 1",
  "term_id": "GO:0042552"
}